{
  "gene": "UniProtKB:Q8NE35",
  "term_id": "GO:0000900",
  "gene_name": "Cytoplasmic polyadenylation element-binding protein 3",
  "term_label": "mRNA regulatory element binding translation repressor activity",
  "gene_symbol": "CPEB3"
}